{
  "gene_name": "Transmembrane protein 255A",
  "term_id": "UNKNOWN:0001",
  "gene": "UniProtKB:Q5JRV8",
  "term_label": "Unknown molecular function",
  "gene_symbol": "TMEM255A"
}